{
  "gene_name": "Vesicle-associated membrane protein 8",
  "term_id": "GO:0035493",
  "term_label": "SNARE complex assembly",
  "gene": "UniProtKB:Q9BV40",
  "gene_symbol": "VAMP8"
}